protocadherin-alpha-v7-protocadherin-gamma-b4 complex [GO:0071191] (cellular component) Also known as: Pcdha7-Pcdhgb2 complex References: PMID:15347688 Relationships: is a type of protocadherin-alpha-protocadherin-gamma complex [GO:0071183] Definition: A protein complex that contains the cell adhesion molecules protocadherin-alpha-v7 and protocadherin-gamma-b4, and is involved in the regulation of protein localization to the plasma membrane.